{
  "gene_symbol": "ZNF622",
  "term_label": "preribosome, large subunit precursor",
  "gene": "UniProtKB:Q969S3",
  "gene_name": "Cytoplasmic 60S subunit biogenesis factor ZNF622",
  "term_id": "GO:0030687"
}